melanization defense response [GO:0035006] (biological process) Also known as: melanization defence response Regulation: regulated by regulation of melanization defense response [GO:0035007]; RO_0002213 by positive regulation of melanization defense response [GO:0035008]; negatively regulated by negative regulation of melanization defense response [GO:0035009] Relationships: is_a GO:0006582; is a type of innate immune response [GO:0045087] Subtypes: melanotic encapsulation of foreign target [GO:0035011] Definition: The blackening of the wounded area of the cuticle or the surface of invading pathogens, parasites or parasitoids, resulting from a proteolytic cascade leading to the de novo synthesis and deposition of melanin. References: PMID:12408809 Sources: GOC:bf